{
  "term_label": "Unknown cellular component",
  "gene_symbol": "M1AP",
  "term_id": "UNKNOWN:0003",
  "gene": "UniProtKB:Q8TC57",
  "gene_name": "Meiosis 1 arrest protein"
}